CD4-positive gamma-delta intraepithelial T cell differentiation [GO:0002306] (biological process) Also known as: CD4-positive, gamma-delta intraepithelial T lymphocyte differentiation, CD4-positive, gamma-delta intraepithelial T-cell differentiation, CD4-positive, gamma-delta intraepithelial T-lymphocyte differentiation, CD4-positive, gamma-delta intraepithelial T cell development Sources: GOC:add, ISBN:0781735149 Relationships: is a type of gamma-delta intraepithelial T cell differentiation [GO:0002304] Note: Note that immunologists typically use the word 'development' to refer to cells of B or T cell lineages undergoing the process that GO describes as 'cell differentiation'. Definition: The process in which a precursor cell type acquires the specialized features of a CD4-positive, gamma-delta intraepithelial T cell. Intraepithelial T cells are found among epithelial cells in mucosal areas and have distinct phenotypes and developmental pathways.